{
  "term_id": "GO:0016567",
  "gene_name": "E3 ubiquitin-protein ligase makorin-1",
  "gene_symbol": "MKRN1",
  "term_label": "protein ubiquitination",
  "gene": "UniProtKB:Q9UHC7"
}